{
  "gene_name": "Calcium_calmodulin-dependent protein kinase II inhibitor 1",
  "gene": "UniProtKB:Q7Z7J9",
  "gene_symbol": "CAMK2N1",
  "term_label": "Unknown cellular component",
  "term_id": "UNKNOWN:0003"
}